{
  "term_id": "GO:0000137",
  "gene": "UniProtKB:Q0D2H9",
  "gene_symbol": "GOLGA8DP",
  "term_label": "Golgi cis cisterna",
  "gene_name": "Putative golgin subfamily A member 8D"
}